{
  "gene_name": "Cation channel sperm-associated auxiliary subunit delta",
  "gene_symbol": "CATSPERD",
  "term_label": "flagellated sperm motility",
  "term_id": "GO:0030317",
  "gene": "UniProtKB:Q86XM0"
}